{
  "term_label": "Unknown cellular component",
  "gene_symbol": "TMEM218",
  "term_id": "UNKNOWN:0003",
  "gene_name": "Transmembrane protein 218",
  "gene": "UniProtKB:A2RU14"
}